{
  "term_id": "GO:0035091",
  "gene_name": "Partitioning defective 3 homolog B",
  "gene_symbol": "PARD3B",
  "gene": "UniProtKB:Q8TEW8",
  "term_label": "phosphatidylinositol binding"
}